{
  "term_label": "signaling receptor binding",
  "gene": "UniProtKB:P08236",
  "term_id": "GO:0005102",
  "gene_symbol": "GUSB",
  "gene_name": "Beta-glucuronidase"
}